{
  "gene": "UniProtKB:P50552",
  "gene_symbol": "VASP",
  "term_label": "profilin binding",
  "gene_name": "Vasodilator-stimulated phosphoprotein",
  "term_id": "GO:0005522"
}